{
  "term_id": "GO:1990246",
  "gene_symbol": "MICU1",
  "gene": "UniProtKB:Q9BPX6",
  "gene_name": "Calcium uptake protein 1, mitochondrial",
  "term_label": "uniplex complex"
}